regulation of miRNA transcription [GO:1902893] (biological process) Definition: Any process that modulates the frequency, rate or extent of microRNA (miRNA) gene transcription. References: PMID:24699545 Sources: GOC:TermGenie, GOC:dph, GOC:kmv, GO_REF:0000058 Also known as: regulation of miRNA gene transcription, regulation of microRNA gene transcription, regulation of pri-miRNA transcription by RNA polymerase II, regulation of pri-miRNA transcription from RNA polymerase II promoter, regulation of primary miRNA gene transcription Relationships: is a type of regulation of DNA-templated transcription [GO:0006355]; is a type of regulation of miRNA metabolic process [GO:2000628]; regulates GO:0061614 Subtypes: negative regulation of miRNA transcription [GO:1902894], positive regulation of miRNA transcription [GO:1902895]